{
  "gene": "UniProtKB:P63162",
  "gene_symbol": "SNRPN",
  "term_id": "GO:0005686",
  "gene_name": "Small nuclear ribonucleoprotein-associated protein N",
  "term_label": "U2 snRNP"
}